positive regulation of establishment of protein localization to mitochondrion [GO:1903749] (biological process) References: PMID:16857185 Sources: GOC:TermGenie, GO_REF:0000058 Definition: Any process that activates or increases the frequency, rate or extent of establishment of protein localization to mitochondrion. Subtypes: positive regulation of protein targeting to mitochondrion [GO:1903955] Also known as: positive regulation of establishment of protein localisation to mitochondrion, positive regulation of establishment of protein localization in mitochondrion, up regulation of establishment of protein localisation to mitochondrion, up regulation of establishment of protein localization in mitochondrion, up regulation of establishment of protein localization to mitochondrion, up-regulation of establishment of protein localisation to mitochondrion, up-regulation of establishment of protein localization in mitochondrion, up-regulation of establishment of protein localization to mitochondrion, upregulation of establishment of protein localisation to mitochondrion, upregulation of establishment of protein localization in mitochondrion, upregulation of establishment of protein localization to mitochondrion, activation of establishment of protein localisation to mitochondrion, activation of establishment of protein localization in mitochondrion, activation of establishment of protein localization to mitochondrion Relationships: is a type of regulation of establishment of protein localization to mitochondrion [GO:1903747]; is a type of positive regulation of establishment of protein localization [GO:1904951]; positively regulates establishment of protein localization to mitochondrion [GO:0072655]